{
  "term_id": "GO:0045944",
  "gene_symbol": "SS18L1",
  "term_label": "positive regulation of transcription by RNA polymerase II",
  "gene_name": "Calcium-responsive transactivator",
  "gene": "UniProtKB:O75177"
}